{
  "term_label": "Unknown molecular function",
  "gene_name": "Transmembrane protein 191C",
  "gene": "UniProtKB:A6NGB0",
  "term_id": "UNKNOWN:0001",
  "gene_symbol": "TMEM191C"
}